{
  "gene_symbol": "CLIC4",
  "gene_name": "Chloride intracellular channel protein 4",
  "term_label": "chloride channel activity",
  "gene": "UniProtKB:Q9Y696",
  "term_id": "GO:0005254"
}